protein disulfide isomerase activity [GO:0003756] (molecular function) Sources: EC:5.3.4.1, GOC:vw, Wikipedia:Protein_disulfide-isomerase#Function Relationships: is a type of GO:0016864; is_a catalytic activity, acting on a protein [GO:0140096] Also known as: disulphide bond formation, protein disulfide-isomerase, protein disulphide isomerase activity, protein thiol-disulfide exchange, protein thiol-disulphide exchange, S-S rearrangase activity, protein cysteine-thiol oxidation Definition: Catalysis of the rearrangement of both intrachain and interchain disulfide bonds in proteins.